mitochondrial respiratory chain complex I assembly [GO:0032981] (biological process) Also known as: mitochondrial NADH dehydrogenase complex (ubiquinone) assembly, mitochondrial complex I assembly Sources: GOC:rph Definition: The aggregation, arrangement and bonding together of a set of components to form mitochondrial respiratory chain complex I. Relationships: is a type of NADH dehydrogenase complex assembly [GO:0010257]; is a type of mitochondrial respiratory chain complex assembly [GO:0033108]